CDP biosynthetic process [GO:0046705] (biological process) Sources: GOC:ai Relationships: is a type of pyrimidine ribonucleoside diphosphate biosynthetic process [GO:0009194]; is a type of pyrimidine ribonucleotide biosynthetic process [GO:0009220]; is a type of GO:0046704 Also known as: CDP anabolism, CDP biosynthesis, CDP formation, CDP synthesis Definition: The chemical reactions and pathways resulting in the formation of CDP, cytidine (5'-)diphosphate.